{
  "gene_name": "Transcription factor p65",
  "gene": "UniProtKB:Q04206",
  "gene_symbol": "RELA",
  "term_id": "GO:0035525",
  "term_label": "NF-kappaB p50/p65 complex"
}